{
  "gene": "UniProtKB:A0A1B0GVN3",
  "gene_name": "Uncharacterized protein C2orf92",
  "gene_symbol": "C2orf92",
  "term_id": "UNKNOWN:0003",
  "term_label": "Unknown cellular component"
}